{
  "gene_name": "Beta-adducin",
  "term_label": "postsynaptic density",
  "term_id": "GO:0014069",
  "gene": "UniProtKB:P35612",
  "gene_symbol": "ADD2"
}